{
  "term_label": "Unknown biological process",
  "gene_symbol": "CYB5B",
  "term_id": "UNKNOWN:0002",
  "gene_name": "Cytochrome b5 type B",
  "gene": "UniProtKB:O43169"
}